{
  "gene": "UniProtKB:Q14140",
  "gene_symbol": "SERTAD2",
  "term_label": "cytoplasm",
  "term_id": "GO:0005737",
  "gene_name": "SERTA domain-containing protein 2"
}